{
  "gene_name": "Glutamate receptor ionotropic, NMDA 3B",
  "term_id": "GO:0008066",
  "gene_symbol": "GRIN3B",
  "gene": "UniProtKB:O60391",
  "term_label": "glutamate receptor activity"
}